growth factor activity [GO:0008083] (molecular function) Sources: ISBN:0815316194 Relationships: is a type of receptor ligand activity [GO:0048018] Note: Also consider annotating to 'receptor agonist activity ; GO:0048018'. Definition: The function that stimulates a cell to grow or proliferate. Most growth factors have other actions besides the induction of cell growth or proliferation.